Rab protein signal transduction [GO:0032482] (biological process) Relationships: is a type of small GTPase-mediated signal transduction [GO:0007264] Regulation: regulated by GO:0032483 Sources: GOC:mah Definition: An intracellular signaling cassette in which a small monomeric GTPase of the Rab subfamily relays a signal.